actin nucleation [GO:0045010] (biological process) Definition: The initial step in the formation of an actin filament, in which actin monomers combine to form a new filament. Nucleation is slow relative to the subsequent addition of more monomers to extend the filament. Also known as: actin filament nucleation Regulation: regulated by regulation of actin nucleation [GO:0051125]; negatively regulated by negative regulation of actin nucleation [GO:0051126]; positively regulated by GO:0051127 Subtypes: GO:0034314, 'de novo' actin filament nucleation [GO:0070060] Sources: ISBN:0815316194 Relationships: is a type of actin filament organization [GO:0007015]